{
  "gene_symbol": "RGS9BP",
  "term_label": "Unknown molecular function",
  "gene_name": "Regulator of G-protein signaling 9-binding protein",
  "gene": "UniProtKB:Q6ZS82",
  "term_id": "UNKNOWN:0001"
}